{
  "gene_symbol": "PAPSS2",
  "term_label": "adenylylsulfate kinase activity",
  "gene": "UniProtKB:O95340",
  "term_id": "GO:0004020",
  "gene_name": "Bifunctional 3'-phosphoadenosine 5'-phosphosulfate synthase 2"
}